{
  "gene": "UniProtKB:Q9HB21",
  "term_id": "GO:0005737",
  "term_label": "cytoplasm",
  "gene_name": "Pleckstrin homology domain-containing family A member 1",
  "gene_symbol": "PLEKHA1"
}